{
  "term_label": "phosphatidylinositol binding",
  "term_id": "GO:0035091",
  "gene": "UniProtKB:Q9H3E2",
  "gene_symbol": "SNX25",
  "gene_name": "Sorting nexin-25"
}